{
  "gene_name": "Transmembrane protease serine 7",
  "term_id": "GO:0008236",
  "gene": "UniProtKB:Q7RTY8",
  "gene_symbol": "TMPRSS7",
  "term_label": "serine-type peptidase activity"
}